{
  "gene_name": "DNA repair protein RAD51 homolog 1",
  "term_label": "DNA strand exchange activity",
  "gene_symbol": "RAD51",
  "term_id": "GO:0000150",
  "gene": "UniProtKB:Q06609"
}